{
  "gene": "UniProtKB:Q9BXR5",
  "term_id": "GO:0038023",
  "term_label": "signaling receptor activity",
  "gene_symbol": "TLR10",
  "gene_name": "Toll-like receptor 10"
}